{
  "term_id": "GO:0004930",
  "gene": "UniProtKB:Q9GZQ6",
  "gene_symbol": "NPFFR1",
  "term_label": "G protein-coupled receptor activity",
  "gene_name": "Neuropeptide FF receptor 1"
}